{
  "gene_name": "E3 ubiquitin-protein ligase RNF113A",
  "gene": "UniProtKB:O15541",
  "term_id": "GO:0004842",
  "gene_symbol": "RNF113A",
  "term_label": "ubiquitin-protein transferase activity"
}